{
  "gene": "UniProtKB:Q96LD1",
  "term_label": "heart contraction",
  "term_id": "GO:0060047",
  "gene_symbol": "SGCZ",
  "gene_name": "Zeta-sarcoglycan"
}